protein transport along microtubule [GO:0098840] (biological process) Also known as: microtubule-based protein transport References: PMID:25987607 Relationships: is a type of intracellular protein transport [GO:0006886]; is a type of transport along microtubule [GO:0010970]; is a type of microtubule-based protein transport [GO:0099118] Definition: The directed movement of a protein along a microtubule, mediated by motor proteins. Subtypes: protein transport along microtubule to cell tip [GO:0099117], axo-dendritic protein transport [GO:0099640], GO:0140210, protein transport along microtubule to spindle pole body [GO:1990852], intramanchette transport [GO:1990953]